{
  "term_id": "GO:0005634",
  "gene": "UniProtKB:Q9UJW8",
  "gene_name": "Zinc finger protein 180",
  "term_label": "nucleus",
  "gene_symbol": "ZNF180"
}